{
  "term_label": "Unknown cellular component",
  "term_id": "UNKNOWN:0003",
  "gene_symbol": "KRTAP9-1",
  "gene_name": "Keratin-associated protein 9-1",
  "gene": "UniProtKB:A8MXZ3"
}